{
  "gene_name": "Cyclin-H",
  "gene_symbol": "CCNH",
  "term_label": "cyclin-dependent protein serine/threonine kinase regulator activity",
  "term_id": "GO:0016538",
  "gene": "UniProtKB:P51946"
}